{
  "gene": "UniProtKB:O15535",
  "gene_name": "Zinc finger and SCAN domain-containing protein 9",
  "term_id": "GO:0000981",
  "term_label": "DNA-binding transcription factor activity, RNA polymerase II-specific",
  "gene_symbol": "ZSCAN9"
}